{
  "term_label": "lysosome",
  "gene_name": "Phospholipase A2 group XV",
  "gene": "UniProtKB:Q8NCC3",
  "gene_symbol": "PLA2G15",
  "term_id": "GO:0005764"
}